{
  "gene": "UniProtKB:O00411",
  "term_id": "GO:0006390",
  "term_label": "mitochondrial transcription",
  "gene_symbol": "POLRMT",
  "gene_name": "DNA-directed RNA polymerase, mitochondrial"
}